{
  "term_label": "exocytosis",
  "term_id": "GO:0006887",
  "gene_name": "Exocyst complex component 3",
  "gene_symbol": "EXOC3",
  "gene": "UniProtKB:O60645"
}